{
  "gene_name": "1,25-dihydroxyvitamin D(3) 24-hydroxylase, mitochondrial",
  "gene_symbol": "CYP24A1",
  "gene": "UniProtKB:Q07973",
  "term_id": "GO:0030342",
  "term_label": "1-alpha,25-dihydroxyvitamin D3 24-hydroxylase activity"
}